{
  "term_id": "UNKNOWN:0002",
  "gene": "UniProtKB:Q6IEG0",
  "gene_name": "U11_U12 small nuclear ribonucleoprotein 48 kDa protein",
  "gene_symbol": "SNRNP48",
  "term_label": "Unknown biological process"
}